cytoplasmic microtubule bundle [GO:1905720] (cellular component) Relationships: is a type of microtubule bundle [GO:0097427]; is part of cytoplasm [GO:0005737] Also known as: microtubule bundle of cytoplasm, microtubule fascicle of cytoplasm References: PMID:11007487, PMID:26124291 Sources: GOC:TermGenie, GO_REF:0000064 Definition: Any microtubule bundle that is part of a cytoplasm.